{
  "term_label": "1-phosphatidylinositol binding",
  "gene": "UniProtKB:Q13492",
  "term_id": "GO:0005545",
  "gene_symbol": "PICALM",
  "gene_name": "Phosphatidylinositol-binding clathrin assembly protein"
}